{
  "term_id": "GO:0008190",
  "gene_symbol": "EIF4EBP1",
  "gene": "UniProtKB:Q13541",
  "gene_name": "Eukaryotic translation initiation factor 4E-binding protein 1",
  "term_label": "eukaryotic initiation factor 4E binding"
}